acrosomal lumen [GO:0043160] (cellular component) Definition: The volume enclosed within the acrosome membrane. Sources: GOC:go_curators Relationships: is a type of secretory granule lumen [GO:0034774]; is a type of lysosomal lumen [GO:0043202]; is part of acrosomal vesicle [GO:0001669]